{
  "gene_name": "Protein FAM228A",
  "gene": "UniProtKB:Q86W67",
  "term_label": "Unknown cellular component",
  "gene_symbol": "FAM228A",
  "term_id": "UNKNOWN:0003"
}